{
  "gene_symbol": "TMEM238",
  "term_id": "UNKNOWN:0003",
  "gene_name": "Transmembrane protein 238",
  "term_label": "Unknown cellular component",
  "gene": "UniProtKB:C9JI98"
}